{
  "gene_symbol": "KRTAP8-1",
  "gene": "UniProtKB:Q8IUC2",
  "term_id": "UNKNOWN:0002",
  "gene_name": "Keratin-associated protein 8-1",
  "term_label": "Unknown biological process"
}